{
  "gene_symbol": "PYDC5",
  "term_label": "Unknown molecular function",
  "term_id": "UNKNOWN:0001",
  "gene": "UniProtKB:W6CW81",
  "gene_name": "Pyrin domain-containing protein 5"
}